lysine-tRNA ligase activity [GO:0004824] (molecular function) Sources: EC:6.1.1.6 Relationships: is a type of aminoacyl-tRNA ligase activity [GO:0004812] Definition: Catalysis of the reaction: ATP + L-lysine + tRNA(Lys) = AMP + diphosphate + L-lysyl-tRNA(Lys). Also known as: lysyl-tRNA synthetase activity, L-lysine-transfer RNA ligase activity, L-lysine:tRNALys ligase (AMP-forming), lysine translase activity, lysine-tRNA synthetase activity, lysyl-transfer RNA synthetase activity, lysyl-transfer ribonucleate synthetase activity